positive regulation of larval somatic muscle development [GO:0062231] (biological process) Definition: Any process that increases the rate, frequency or extent of larval somatic muscle development. Relationships: is a type of positive regulation of somatic muscle development [GO:0062224]; is a type of regulation of larval somatic muscle development [GO:0062229]; positively regulates larval somatic muscle development [GO:0007526] References: PMID:16643882, PMID:25758712